{
  "term_label": "cell adhesion molecule binding",
  "gene": "UniProtKB:Q9Y5E9",
  "gene_symbol": "PCDHB14",
  "term_id": "GO:0050839",
  "gene_name": "Protocadherin beta-14"
}